1,5-anhydro-D-fructose reductase activity [GO:0050571] (molecular function) Definition: Catalysis of the reaction: 1,5-anhydro-D-glucitol + NADP+ = 1,5-anhydro-D-fructose + H+ + NADPH. Sources: EC:1.1.1.263, RHEA:20665 Also known as: 1,5-anhydro-D-glucitol:NADP+ oxidoreductase activity, AF reductase activity Relationships: is a type of oxidoreductase activity, acting on the CH-OH group of donors, NAD or NADP as acceptor [GO:0016616]